{
  "gene_symbol": "APOL3",
  "term_label": "Unknown biological process",
  "term_id": "UNKNOWN:0002",
  "gene_name": "Apolipoprotein L3",
  "gene": "UniProtKB:O95236"
}